{
  "gene_symbol": "AP5M1",
  "gene_name": "AP-5 complex subunit mu-1",
  "term_label": "cytosol",
  "term_id": "GO:0005829",
  "gene": "UniProtKB:Q9H0R1"
}